NADPH peroxidase activity [GO:0050137] (MF) Also known as: NADP peroxidase activity, NADPH:hydrogen-peroxide oxidoreductase activity, TPN peroxidase activity, TPNH peroxidase activity, nicotinamide adenine dinucleotide phosphate peroxidase activity, triphosphopyridine nucleotide peroxidase activity Relationships: is a type of GO:0004601 Definition: Catalysis of the reaction: H2O2 + H+ + NADPH = 2 H2O + NADP+. Sources: EC:1.11.1.2, RHEA:15173